diphosphate-glycerol phosphotransferase activity [GO:0047331] (molecular function) Sources: EC:2.7.1.79, RHEA:13689 Relationships: is a type of kinase activity [GO:0016301]; is a type of GO:0016773 Definition: Catalysis of the reaction: glycerol + diphosphate = glycerol 1-phosphate + H+ + phosphate. Also known as: PPi-glycerol phosphotransferase activity, diphosphate:glycerol 1-phosphotransferase activity, pyrophosphate--glycerol phosphotransferase activity